{
  "gene_symbol": "C1orf141",
  "term_id": "UNKNOWN:0003",
  "gene_name": "Uncharacterized protein C1orf141",
  "term_label": "Unknown cellular component",
  "gene": "UniProtKB:Q5JVX7"
}